{
  "gene_name": "Oxoeicosanoid receptor 1",
  "gene": "UniProtKB:Q8TDS5",
  "gene_symbol": "OXER1",
  "term_id": "GO:0005886",
  "term_label": "plasma membrane"
}